symbiont entry into host cell via permeabilization of host membrane [GO:0140267] (biological process) Definition: The entry of a symbiont into the cytoplasm of a host cell, triggered by an interaction between the bilayer of a host membrane and a membrane-penetration symbiont protein. This process mediates the entry of some non-enveloped virus into host cells, and results in the release of the virus contents into the host cell cytoplasm. References: PMID:20427561, PMID:25055856 Sources: VZ:985 Relationships: is a type of symbiont-mediated perturbation of host membrane [GO:0141171]; BFO_0000050 symbiont entry into host cell [GO:0046718] Also known as: viral entry via permeabilization of host membrane Subtypes: symbiont entry into host cell via permeabilization of endosomal membrane [GO:0099006], symbiont entry into host cell via permeabilization of inner membrane [GO:0099008]